{
  "gene_name": "1-acylglycerol-3-phosphate O-acyltransferase ABHD5",
  "gene": "UniProtKB:Q8WTS1",
  "term_id": "GO:0005811",
  "term_label": "lipid droplet",
  "gene_symbol": "ABHD5"
}